{
  "gene_symbol": "ZNF700",
  "gene_name": "Zinc finger protein 700",
  "term_label": "nucleus",
  "gene": "UniProtKB:Q9H0M5",
  "term_id": "GO:0005634"
}